{
  "term_label": "Unknown molecular function",
  "term_id": "UNKNOWN:0001",
  "gene_name": "Late cornified envelope protein 1E",
  "gene": "UniProtKB:Q5T753",
  "gene_symbol": "LCE1E"
}